positive regulation of substance P secretion, neurotransmission [GO:1904496] (biological process) Definition: Any process that activates or increases the frequency, rate or extent of substance P secretion, neurotransmission. Also known as: up regulation of substance P secretion, neurotransmission, up-regulation of substance P secretion, neurotransmission, upregulation of substance P secretion, neurotransmission, activation of substance P secretion, neurotransmission References: PMID:15292051 Sources: GOC:TermGenie, GO_REF:0000058 Relationships: is a type of positive regulation of neurotransmitter secretion [GO:0001956]; is a type of positive regulation of substance P secretion [GO:1904460]; is a type of regulation of substance P secretion, neurotransmission [GO:1904494]; positively regulates substance P secretion, neurotransmission [GO:1990793]